adenosylmethionine-8-amino-7-oxononanoate transaminase activity [GO:0004015] (molecular function) Definition: Catalysis of the reaction: 8-amino-7-oxononanoate + S-adenosyl-L-methionine(1+) = 7,8-diaminononanoate + S-adenosyl-4-methylthio-2-oxobutanoate. Sources: EC:2.6.1.62, RHEA:16861 Relationships: is a type of GO:0008483 Also known as: adenosyl methionine-8-amino-7-oxononanoate transaminase activity, adenosylmethionine-8-amino-7-oxononanoate aminotransferase activity, 7,8-diamino-pelargonic acid aminotransferase activity, 7,8-diaminonanoate transaminase activity, 7,8-diaminononanoate aminotransferase activity, 7,8-diaminononanoate transaminase activity, 7,8-diaminopelargonic acid aminotransferase activity, 7-keto-8-aminopelargonic acid, 7-keto-8-aminopelargonic acid aminotransferase activity, DAPA aminotransferase activity, DAPA transaminase activity, S-adenosyl-L-methionine:8-amino-7-oxononanoate aminotransferase activity, adenosylmethionine--8-amino-7-oxononanoate aminotransferase activity, diaminopelargonate synthase activity